{
  "gene": "UniProtKB:Q969H6",
  "term_label": "multimeric ribonuclease P complex",
  "term_id": "GO:0030681",
  "gene_name": "Ribonuclease P_MRP protein subunit POP5",
  "gene_symbol": "POP5"
}